{
  "gene_symbol": "BMS1",
  "gene_name": "Ribosome biogenesis protein BMS1 homolog",
  "term_label": "nucleolus",
  "gene": "UniProtKB:Q14692",
  "term_id": "GO:0005730"
}